{
  "gene": "UniProtKB:P14651",
  "term_id": "GO:0000978",
  "term_label": "RNA polymerase II cis-regulatory region sequence-specific DNA binding",
  "gene_name": "Homeobox protein Hox-B3",
  "gene_symbol": "HOXB3"
}